{
  "gene_symbol": "SLC36A2",
  "gene_name": "Proton-coupled amino acid transporter 2",
  "gene": "UniProtKB:Q495M3",
  "term_id": "GO:0005774",
  "term_label": "vacuolar membrane"
}